retromer, tubulation complex [GO:0030905] (cellular component) Also known as: SNX-BAR dimer, heterodimeric membrane-deforming retromer subcomplex, retromer complex, outer shell Definition: The dimeric subcomplex of the retromer, believed to be peripherally associated with the membrane. This dimeric complex is responsible for remodeling endosomal membranes to form a tube-structure to which cargo molecules are selected for recycling. The budding yeast complex comprises Vps5p and Vps17p, and may contain multiple copies of a Vps5p/Vps17p dimer. The mammalian complex contains SNX1 or SNX2 dimerized with SNX5 or SNX6. References: PMID:26220253, PMID:9700157 Sources: GOC:bf Relationships: is a type of membrane protein complex [GO:0098796]; is part of GO:0030904